Entner-Doudoroff pathway through 6-phosphogluconate [GO:0009255] (biological process) Relationships: is a type of GO:0019682; is_a Entner-Doudoroff pathway [GO:0061678]; has part phosphogluconate dehydratase activity [GO:0004456]; has part 2-dehydro-3-deoxy-phosphogluconate aldolase activity [GO:0008675] Definition: A pathway that converts a carbohydrate to pyruvate and glyceraldehyde-3 phosphate by producing 6-phosphogluconate and then dehydrating it. References: PMID:12921356, PMID:12981024 Sources: GOC:jl, MetaCyc:PWY-8004